{
  "term_label": "Unknown molecular function",
  "gene": "UniProtKB:Q8TB05",
  "gene_symbol": "UBALD1",
  "gene_name": "UBA-like domain-containing protein 1",
  "term_id": "UNKNOWN:0001"
}